{
  "gene_name": "Opioid growth factor receptor-like protein 1",
  "term_id": "UNKNOWN:0001",
  "gene_symbol": "OGFRL1",
  "term_label": "Unknown molecular function",
  "gene": "UniProtKB:Q5TC84"
}